{
  "gene": "UniProtKB:Q96C03",
  "term_id": "GO:0090141",
  "term_label": "positive regulation of mitochondrial fission",
  "gene_name": "Mitochondrial dynamics protein MID49",
  "gene_symbol": "MIEF2"
}